{
  "gene": "UniProtKB:Q7Z449",
  "term_id": "GO:0005737",
  "gene_name": "Cytochrome P450 2U1",
  "gene_symbol": "CYP2U1",
  "term_label": "cytoplasm"
}